{
  "gene_symbol": "KRT34",
  "term_id": "GO:0045095",
  "gene_name": "Keratin, type I cuticular Ha4",
  "gene": "UniProtKB:O76011",
  "term_label": "keratin filament"
}